{
  "gene_symbol": "RAB24",
  "gene": "UniProtKB:Q969Q5",
  "gene_name": "Ras-related protein Rab-24",
  "term_id": "GO:0005768",
  "term_label": "endosome"
}